{
  "gene_symbol": "LEP",
  "gene": "UniProtKB:P41159",
  "term_label": "negative regulation of appetite by leptin-mediated signaling pathway",
  "term_id": "GO:0038108",
  "gene_name": "Leptin"
}